{
  "gene": "UniProtKB:Q8NH73",
  "gene_name": "Olfactory receptor 4S2",
  "gene_symbol": "OR4S2",
  "term_label": "plasma membrane",
  "term_id": "GO:0005886"
}